{
  "gene_symbol": "CCDC87",
  "term_id": "UNKNOWN:0002",
  "gene": "UniProtKB:Q9NVE4",
  "term_label": "Unknown biological process",
  "gene_name": "Coiled-coil domain-containing protein 87"
}